{
  "gene_symbol": "DHRS7C",
  "gene": "UniProtKB:A6NNS2",
  "gene_name": "Dehydrogenase_reductase SDR family member 7C",
  "term_id": "UNKNOWN:0003",
  "term_label": "Unknown cellular component"
}